{
  "gene": "UniProtKB:Q9NWW6",
  "term_label": "nicotinate riboside kinase activity",
  "gene_symbol": "NMRK1",
  "gene_name": "Nicotinamide riboside kinase 1",
  "term_id": "GO:0061769"
}